{
  "term_label": "nucleus",
  "gene": "UniProtKB:P25788",
  "term_id": "GO:0005634",
  "gene_symbol": "PSMA3",
  "gene_name": "Proteasome subunit alpha type-3"
}